regulation of laminaritriose transport [GO:1900303] (biological process) Subtypes: negative regulation of laminaritriose transport [GO:1900304], positive regulation of laminaritriose transport [GO:1900305] Sources: GOC:TermGenie, GOC:mengo_curators Relationships: is a type of regulation of transport [GO:0051049]; RO_0002211 GO:2001097 Definition: Any process that modulates the frequency, rate or extent of laminaritriose transport.